{
  "term_id": "GO:0000776",
  "gene_symbol": "DCTN1",
  "gene_name": "Dynactin subunit 1",
  "gene": "UniProtKB:Q14203",
  "term_label": "kinetochore"
}